{
  "gene_name": "Mothers against decapentaplegic homolog 1",
  "term_label": "regulation of transcription by RNA polymerase II",
  "gene_symbol": "SMAD1",
  "term_id": "GO:0006357",
  "gene": "UniProtKB:Q15797"
}